{
  "term_id": "GO:0010312",
  "gene_name": "Calcium_manganese antiporter SLC30A10",
  "term_label": "detoxification of zinc ion",
  "gene": "UniProtKB:Q6XR72",
  "gene_symbol": "SLC30A10"
}